{
  "term_id": "UNKNOWN:0001",
  "term_label": "Unknown molecular function",
  "gene": "UniProtKB:Q9UKD2",
  "gene_symbol": "MRTO4",
  "gene_name": "mRNA turnover protein 4 homolog"
}